{
  "term_id": "GO:0005634",
  "term_label": "nucleus",
  "gene": "UniProtKB:Q71DI3",
  "gene_name": "Histone H3.2",
  "gene_symbol": "H3C13"
}